{
  "term_label": "calcitonin receptor binding",
  "term_id": "GO:0031716",
  "gene": "UniProtKB:P10092",
  "gene_name": "Calcitonin gene-related peptide 2",
  "gene_symbol": "CALCB"
}